regulation of cholangiocyte apoptotic process [GO:1904192] (biological process) Relationships: is a type of regulation of epithelial cell apoptotic process [GO:1904035]; regulates cholangiocyte apoptotic process [GO:1902488] Definition: Any process that modulates the frequency, rate or extent of cholangiocyte apoptotic process. References: PMID:24498161 Sources: GOC:TermGenie, GO_REF:0000058 Subtypes: GO:1904193, positive regulation of cholangiocyte apoptotic process [GO:1904194] Also known as: regulation of epithelial cell of bile duct apoptotic process, regulation of cholangiocyte apoptosis, regulation of epithelial cell of bile duct apoptosis